pancreatic polypeptide secretion [GO:0036322] (biological process) References: PMID:12730894 Sources: GOC:cjm, Wikipedia:Pancreatic_polypeptide Relationships: is a type of peptide hormone secretion [GO:0030072] Definition: The regulated release of pancreatic polypeptide (PP) from a cell. Pancreatic polypeptide is a 36 amino acid polypeptide secreted by islets of Langerhans cells in the pancreas. Also known as: PP secretion